{
  "term_label": "RNA polymerase II cis-regulatory region sequence-specific DNA binding",
  "term_id": "GO:0000978",
  "gene": "UniProtKB:P0CG00",
  "gene_symbol": "ZSCAN5DP",
  "gene_name": "Putative zinc finger and SCAN domain-containing protein 5D"
}